{
  "gene_symbol": "PURA",
  "gene": "UniProtKB:Q00577",
  "term_label": "nucleus",
  "term_id": "GO:0005634",
  "gene_name": "Transcriptional activator protein Pur-alpha"
}